{
  "term_id": "UNKNOWN:0002",
  "gene": "UniProtKB:Q8WU49",
  "term_label": "Unknown biological process",
  "gene_name": "Uncharacterized protein C7orf33",
  "gene_symbol": "C7orf33"
}